establishment or maintenance of bipolar cell polarity [GO:0061245] (biological process) Regulation: RO_0002211 by regulation of establishment or maintenance of bipolar cell polarity [GO:2000099] Subtypes: establishment or maintenance of apical/basal cell polarity [GO:0035088], establishment or maintenance of bipolar cell polarity regulating cell shape [GO:0061246] Sources: GOC:dph, GOC:vw Relationships: is a type of establishment or maintenance of cell polarity [GO:0007163] Definition: Any cellular process that results in the specification, formation or maintenance of a bipolar intracellular organization or cell growth patterns.